{
  "gene_symbol": "RASSF1",
  "term_label": "Unknown molecular function",
  "gene_name": "Ras association domain-containing protein 1",
  "term_id": "UNKNOWN:0001",
  "gene": "UniProtKB:Q9NS23"
}